{
  "gene_name": "Small integral membrane protein 31",
  "term_id": "UNKNOWN:0001",
  "gene": "UniProtKB:A0A1B0GVY4",
  "gene_symbol": "SMIM31",
  "term_label": "Unknown molecular function"
}